{
  "term_id": "GO:0000922",
  "gene": "UniProtKB:O95835",
  "gene_name": "Serine_threonine-protein kinase LATS1",
  "term_label": "spindle pole",
  "gene_symbol": "LATS1"
}